regulation of synaptic vesicle priming [GO:0010807] (biological process) References: PMID:15489511 Sources: GOC:dph, GOC:kmv, GOC:tb Relationships: is a type of regulation of protein-containing complex assembly [GO:0043254]; regulates GO:0016082 Subtypes: positive regulation of synaptic vesicle priming [GO:0010808], negative regulation of synaptic vesicle priming [GO:0010809] Definition: Any process that modulates the frequency, rate or extent of synaptic vesicle priming. Synaptic vesicle priming is the formation of SNARE-containing complexes, bringing synaptic vesicle membrane and plasma membranes into close proximity and thereby facilitating membrane fusion.